{
  "term_id": "UNKNOWN:0003",
  "gene": "UniProtKB:Q96BJ8",
  "gene_name": "Engulfment and cell motility protein 3",
  "term_label": "Unknown cellular component",
  "gene_symbol": "ELMO3"
}